{
  "gene_symbol": "ENTR1",
  "gene_name": "Endosome-associated-trafficking regulator 1",
  "term_id": "GO:0045724",
  "term_label": "positive regulation of cilium assembly",
  "gene": "UniProtKB:Q96C92"
}